positive regulation of maltopentaose transport [GO:1900317] (biological process) Definition: Any process that activates or increases the frequency, rate or extent of maltopentaose transport. Sources: GOC:TermGenie, GOC:mengo_curators Also known as: up regulation of maltopentaose transport, up-regulation of maltopentaose transport, upregulation of maltopentaose transport, activation of maltopentaose transport Relationships: is a type of GO:1900315; is a type of positive regulation of pentasaccharide transport [GO:1900362]; positively regulates GO:2001101